lateral geniculate nucleus development [GO:0021771] (biological process) Also known as: LGN development Relationships: is a type of GO:0048857; is part of GO:0021794 Sources: GOC:cls, GOC:dgh, GOC:dph, GOC:jid, GO_REF:0000021 Definition: The progression of the lateral geniculate nucleus over time from its initial formation until its mature state. The lateral geniculate nucleus is the primary processor of visual information received from the retina.